{
  "gene_name": "Pyroglutamyl-peptidase 1-like protein",
  "gene_symbol": "PGPEP1L",
  "term_id": "UNKNOWN:0003",
  "term_label": "Unknown cellular component",
  "gene": "UniProtKB:A6NFU8"
}